[3-methyl-2-oxobutanoate dehydrogenase (lipoamide)]-phosphatase activity [GO:0047385] (molecular function) Relationships: is a type of phosphoprotein phosphatase activity [GO:0004721] Also known as: branched-chain 2-keto acid dehydrogenase phosphatase activity, branched-chain alpha-keto acid dehydrogenase phosphatase, branched-chain oxo-acid dehydrogenase phosphatase activity Definition: Catalysis of the reaction: H2O + O-phospho-L-seryl-[3-methyl-2-oxobutanoate dehydrogenase] = L-seryl-[3-methyl-2-oxobutanoate dehydrogenase] + phosphate. Sources: EC:3.1.3.52